UDP-2-acetamido-4-amino-2,4,6-trideoxyglucose transaminase activity [GO:0047302] (molecular function) Relationships: is a type of transaminase activity [GO:0008483] References: PMID:16286454 Sources: RHEA:31663 Also known as: UDP-4-amino-2-acetamido-2,4,6-trideoxyglucose aminotransferase activity, UDP-4-amino-2-acetamido-2,4,6-trideoxyglucose transaminase activity, UDP-2-acetamido-4-amino-2,4,6-trideoxyglucose:2-oxoglutarate aminotransferase activity, uridine diphospho-4-amino-2-acetamido-2,4,6-trideoxyglucose aminotransferase activity Definition: Catalysis of the reaction: 2-oxoglutarate + UDP-2-acetamido-4-amino-2,4,6-trideoxy-D-glucose = L-glutamate + UDP-2-acetamido-4-dehydro-2,6-dideoxy-beta-D-glucose.